interleukin-2 production [GO:0032623] (biological process) Also known as: IL-2 production, interleukin-2 biosynthetic process, interleukin-2 secretion Sources: GOC:mah Relationships: is a type of cytokine production [GO:0001816] Regulation: RO_0002211 by GO:0032663; RO_0002212 by negative regulation of interleukin-2 production [GO:0032703]; positively regulated by GO:0032743 Definition: The appearance of interleukin-2 due to biosynthesis or secretion following a cellular stimulus, resulting in an increase in its intracellular or extracellular levels.